{
  "gene_name": "C-Jun-amino-terminal kinase-interacting protein 1",
  "term_id": "GO:0008432",
  "gene_symbol": "MAPK8IP1",
  "term_label": "JUN kinase binding",
  "gene": "UniProtKB:Q9UQF2"
}